sporocarp development involved in sexual reproduction [GO:0000909] (biological process) Definition: The process whose specific outcome is the progression of a fruiting body organ over time, from its formation to the mature structure. The fruiting body is a spore bearing structure. In fungi, the sporocarp (also known as fruiting body) is a multicellular structure on which spore-producing structures, such as basidia or asci, are borne. The fruiting body is part of the sexual phase of a fungal life cycle, with the rest of the life cycle being characterized by vegetative mycelial growth. The sporocarp of a basidiomycete is known as a basidiocarp, while the fruiting body of an ascomycete is known as an ascocarp. A significant range of different shapes and morphologies is found in both basidiocarps and ascocarps; these features play an important role in the identification and taxonomy of fungi. Sources: GOC:clt, GOC:mtg_sensu Also known as: fruiting body development involved in sexual reproduction, fruiting body formation involved in sexual reproduction, ascus development, perfect stage fruiting body development Relationships: is a type of sporocarp development [GO:0030584]; is part of GO:0019953 Subtypes: GO:0070791 Regulation: regulated by GO:1902058; negatively regulated by negative regulation of sporocarp development involved in sexual reproduction [GO:1902059]; positively regulated by GO:1902060